{
  "term_label": "Unknown biological process",
  "gene_name": "Spermatogenesis-associated protein 31D4",
  "term_id": "UNKNOWN:0002",
  "gene": "UniProtKB:Q6ZUB0",
  "gene_symbol": "SPATA31D4"
}